{
  "term_label": "GABA-A receptor activity",
  "gene": "UniProtKB:P28476",
  "gene_name": "Gamma-aminobutyric acid receptor subunit rho-2",
  "gene_symbol": "GABRR2",
  "term_id": "GO:0004890"
}